{
  "term_label": "cis-Golgi network",
  "gene_symbol": "GOLGA8N",
  "gene": "UniProtKB:F8WBI6",
  "gene_name": "Golgin subfamily A member 8N",
  "term_id": "GO:0005801"
}